virus tail, fiber [GO:0098024] (cellular component) Also known as: bacteriophage tail fiber Definition: The fibrous region of the virus tail used to scan, recognize and attach to the host cell. Note: For tailed bacteriophages, fibers typically bind to particular Lipopolysaccharide (LPS), polysaccharide or protein receptors on the cell surface. Relationships: is a type of virion component [GO:0044423]; is part of virus tail [GO:0098015] Sources: GOC:bm, VZ:4416